{
  "term_label": "endoplasmic reticulum membrane",
  "term_id": "GO:0005789",
  "gene_name": "Probable cation-transporting ATPase 13A4",
  "gene": "UniProtKB:Q4VNC1",
  "gene_symbol": "ATP13A4"
}